bacterial-type flagellum hook-filament junction [GO:0009422] (cellular component) References: PMID:10572114, PMID:12624192 Sources: GOC:cilia, GOC:mah, GOC:mtg_sensu Definition: The region of the bacterial-type flagellum where the hook and filament meet. Also known as: flagellar hook-filament junction Relationships: is a type of cellular anatomical structure [GO:0110165]; is part of GO:0009288